{
  "gene": "UniProtKB:Q7L190",
  "term_label": "nucleus",
  "gene_symbol": "DPPA4",
  "gene_name": "Developmental pluripotency-associated protein 4",
  "term_id": "GO:0005634"
}